arterial endothelial cell differentiation [GO:0060842] (biological process) Definition: The process in which a relatively unspecialized endothelial cell acquires specialized features of an arterial endothelial cell, a thin flattened cell that lines the inside surfaces of arteries. Relationships: is a type of blood vessel endothelial cell differentiation [GO:0060837] Sources: GOC:dph, GOC:sdb_2009, GOC:tb